{
  "gene_name": "Inactive glutathione hydrolase 2",
  "term_label": "glutathione catabolic process",
  "gene": "UniProtKB:P36268",
  "term_id": "GO:0006751",
  "gene_symbol": "GGT2P"
}